tryptophan synthase activity [GO:0004834] (molecular function) Relationships: is a type of GO:0016836; is part of L-tryptophan biosynthetic process [GO:0000162] Also known as: L-serine hydro-lyase (adding indoleglycerol-phosphate), L-serine hydro-lyase [adding 1-C-(indol-3-yl)glycerol 3-phosphate; L-tryptophan and glyceraldehyde-3-phosphate-forming], L-tryptophan synthetase activity, indoleglycerol phosphate aldolase activity, tryptophan desmolase activity, tryptophan synthetase activity Definition: Catalysis of the reaction: L-serine + (1S,2R)-1-C-(indol-3-yl)glycerol 3-phosphate = L-tryptophan + glyceraldehyde 3-phosphate + H2O. Sources: RHEA:10532